{
  "gene_symbol": "WNK1",
  "term_id": "GO:0004674",
  "gene": "UniProtKB:Q9H4A3",
  "gene_name": "Serine_threonine-protein kinase WNK1",
  "term_label": "protein serine/threonine kinase activity"
}